{
  "gene_symbol": "GP2",
  "gene": "UniProtKB:P55259",
  "gene_name": "Pancreatic secretory granule membrane major glycoprotein GP2",
  "term_id": "GO:1990266",
  "term_label": "neutrophil migration"
}